{
  "term_label": "Unknown molecular function",
  "term_id": "UNKNOWN:0001",
  "gene": "UniProtKB:Q14315",
  "gene_name": "Filamin-C",
  "gene_symbol": "FLNC"
}